cellular response to ionomycin [GO:1904637] (biological process) Relationships: is a type of cellular response to ether [GO:0071362]; is a type of GO:0071398; is a type of response to ionomycin [GO:1904636] References: PMID:17516843 Sources: GOC:TermGenie, GO_REF:0000071 Definition: Any process that results in a change in state or activity of a cell (in terms of movement, secretion, enzyme production, gene expression, etc.) as a result of an ionomycin stimulus.